interleukin-20 receptor complex [GO:0030876] (CC) Definition: A protein complex composed of an alpha and a beta receptor subunit and an interleukin ligand. In human, Interleukin-19, -20 and -24 bind IL20RA/IL20RB receptor subunits and Interleukin-20 and -24 bind IL22RA1/IL20RB receptor subunits. Also known as: IL-20 receptor complex References: PMID:12351624 Relationships: is a type of plasma membrane signaling receptor complex [GO:0098802]